prenol biosynthetic process [GO:0016091] (biological process) Relationships: is a type of isoprenoid biosynthetic process [GO:0008299]; is a type of GO:0046165; is a type of olefinic compound biosynthetic process [GO:0120255] Definition: The chemical reactions and pathways resulting in the formation of prenols, isoprenoids of general formula (H-CH2-C(CH3)=CH-CH2-)n-OH, any primary monohydroxy alcohol whose carbon skeleton consists of two or more isoprenoid residues linked head to tail. Sources: GOC:go_curators Also known as: prenol anabolism, prenol biosynthesis, prenol formation, prenol synthesis